{
  "term_id": "GO:0030674",
  "gene": "UniProtKB:Q13418",
  "term_label": "protein-macromolecule adaptor activity",
  "gene_symbol": "ILK",
  "gene_name": "Integrin-linked protein kinase"
}